{
  "term_id": "GO:0043235",
  "gene": "UniProtKB:P35968",
  "gene_symbol": "KDR",
  "gene_name": "Vascular endothelial growth factor receptor 2",
  "term_label": "receptor complex"
}